{
  "gene_symbol": "DOP1A",
  "term_label": "Unknown molecular function",
  "gene_name": "Protein dopey-1",
  "term_id": "UNKNOWN:0001",
  "gene": "UniProtKB:Q5JWR5"
}